{
  "term_label": "desmosome",
  "gene_symbol": "DSG3",
  "gene": "UniProtKB:P32926",
  "gene_name": "Desmoglein-3",
  "term_id": "GO:0030057"
}